{
  "gene_name": "Neuropeptides B_W receptor type 2",
  "term_id": "GO:0043005",
  "gene_symbol": "NPBWR2",
  "gene": "UniProtKB:P48146",
  "term_label": "neuron projection"
}